{
  "term_label": "DNA repair",
  "gene": "UniProtKB:Q5VVX9",
  "term_id": "GO:0006281",
  "gene_name": "Ubiquitin-conjugating enzyme E2 U",
  "gene_symbol": "UBE2U"
}